glycerol-3-phosphate O-acyltransferase activity [GO:0004366] (molecular function) Relationships: is a type of GO:0008374 Also known as: 3-glycerophosphate acyltransferase activity, ACP:sn-glycerol-3-phosphate acyltransferase activity, acyl-CoA:sn-glycerol-3-phosphate 1-O-acyltransferase activity, alpha-glycerophosphate acyltransferase activity, glycerol 3-phosphate acyltransferase activity, glycerol phosphate acyltransferase activity, glycerol phosphate transacylase activity, glycerophosphate acyltransferase activity, glycerophosphate transacylase activity, sn-glycerol 3-phosphate acyltransferase activity, sn-glycerol-3-phosphate acyltransferase activity Sources: RHEA:15325 Definition: Catalysis of the reaction: an acyl-CoA + sn-glycerol 3-phosphate = a 1-acyl-sn-glycero-3-phosphate + CoA.